{
  "term_id": "GO:1990756",
  "term_label": "ubiquitin-like ligase-substrate adaptor activity",
  "gene_name": "PRAME family member 27",
  "gene": "UniProtKB:A3QJZ7",
  "gene_symbol": "PRAMEF27"
}